positive regulation of endosome to plasma membrane protein transport [GO:1905751] (biological process) Also known as: up regulation of endosome to plasma membrane protein transport, up-regulation of endosome to plasma membrane protein transport, upregulation of endosome to plasma membrane protein transport, activation of endosome to plasma membrane protein transport Relationships: is a type of positive regulation of intracellular protein transport [GO:0090316]; is_a positive regulation of protein localization to plasma membrane [GO:1903078]; is a type of regulation of endosome to plasma membrane protein transport [GO:1905749]; is a type of positive regulation of endocytic recycling [GO:2001137]; positively regulates GO:0099638 Definition: Any process that activates or increases the frequency, rate or extent of endosome to plasma membrane protein transport. References: PMID:22869721 Sources: GOC:TermGenie, GO_REF:0000058